{
  "gene": "UniProtKB:Q5T8I9",
  "gene_symbol": "HENMT1",
  "gene_name": "Small RNA 2'-O-methyltransferase",
  "term_label": "O-methyltransferase activity",
  "term_id": "GO:0008171"
}